{
  "term_label": "regulation of translation at presynapse, modulating synaptic transmission",
  "gene_name": "RNA-binding protein FXR1",
  "gene_symbol": "FXR1",
  "gene": "UniProtKB:P51114",
  "term_id": "GO:0099577"
}